mRNA alternative polyadenylation [GO:0110104] (biological process) Relationships: is a type of mRNA 3'-end processing [GO:0031124] Regulation: regulated by GO:0140408; positively regulated by GO:0140409 References: PMID:28453393, PMID:29276085 Sources: GOC:ans Definition: The process of generating multiple mRNA molecules with variable 3'-end length formation from a given pre-mRNA by differential use of cleavage and polyadenylation signals (pA signals).